{
  "gene_symbol": "OR52P1",
  "term_label": "olfactory receptor activity",
  "term_id": "GO:0004984",
  "gene": "UniProtKB:Q8NH57",
  "gene_name": "Olfactory receptor 52P1"
}